{
  "term_id": "GO:0031012",
  "gene_symbol": "ADAMTS4",
  "gene_name": "A disintegrin and metalloproteinase with thrombospondin motifs 4",
  "term_label": "extracellular matrix",
  "gene": "UniProtKB:O75173"
}